negative regulation of plant epidermal cell differentiation [GO:1903889] (biological process) References: PMID:123345 Sources: GOC:TermGenie, GO_REF:0000058 Relationships: is a type of negative regulation of cell differentiation [GO:0045596]; is a type of regulation of plant epidermal cell differentiation [GO:1903888]; negatively regulates plant epidermal cell differentiation [GO:0090627] Also known as: down regulation of plant epidermal cell differentiation, down-regulation of plant epidermal cell differentiation, downregulation of plant epidermal cell differentiation, inhibition of plant epidermal cell differentiation Subtypes: negative regulation of atrichoblast fate specification [GO:0010060], GO:0010062 Definition: Any process that stops, prevents or reduces the frequency, rate or extent of plant epidermal cell differentiation.